{
  "term_id": "GO:0005634",
  "gene_symbol": "CDX4",
  "term_label": "nucleus",
  "gene": "UniProtKB:O14627",
  "gene_name": "Homeobox protein CDX-4"
}